{
  "term_label": "spindle",
  "term_id": "GO:0005819",
  "gene_symbol": "SAC3D1",
  "gene": "UniProtKB:A6NKF1",
  "gene_name": "SAC3 domain-containing protein 1"
}